cytoproct [GO:0031911] (cellular component) Relationships: is a type of cellular anatomical structure [GO:0110165]; is part of plasma membrane [GO:0005886] Definition: Stable, specialized structure for extrusion of waste by the cell into the surrounding medium. References: PMID:10503189, PMID:23317460, PMID:27889663